selenium compound metabolic process [GO:0001887] (biological process) Definition: The chemical reactions and pathways involving compounds that contain selenium, such as selenocysteine. Also known as: selenium compound metabolism, selenium metabolic process, selenium metabolism Relationships: is a type of GO:0008152 Subtypes: tRNA seleno-modification [GO:0070329] References: PMID:12730456